guanylate cyclase activator activity [GO:0030250] (molecular function) Subtypes: calcium sensitive guanylate cyclase activator activity [GO:0008048] Relationships: is a type of cyclase activator activity [GO:0010853]; is a type of GO:0030249; positively regulates guanylate cyclase activity [GO:0004383] Sources: GOC:mah Also known as: guanylin Definition: Binds to and increases the activity of guanylate cyclase.